{
  "gene": "UniProtKB:O75928",
  "gene_name": "E3 SUMO-protein ligase PIAS2",
  "term_label": "transcription coregulator activity",
  "term_id": "GO:0003712",
  "gene_symbol": "PIAS2"
}